negative regulation of mitotic spindle pole body separation [GO:0010697] (biological process) Definition: Any process that decreases the rate, frequency or extent of the process involving the release of duplicated mitotic spindle pole bodies (SPBs) and their migration away from each other within the nuclear membrane. References: PMID:16792804, PMID:18500339 Sources: GOC:dph, GOC:tb Also known as: negative regulation of SPB separation Relationships: is a type of GO:0010695; is a type of negative regulation of cell cycle process [GO:0010948]; negatively regulates initial mitotic spindle pole body separation [GO:0000073]